U11 snRNP [GO:0005692] (cellular component) Sources: GOC:krc, GOC:mah, ISBN:0879695897 Relationships: is a type of GO:0097525 Definition: A ribonucleoprotein complex that contains small nuclear RNA U11, a heptameric ring of Sm proteins, as well as several proteins that are unique to the U11 snRNP, most of which remain associated with the U11 snRNA both while the U11 snRNP is free or assembled into a series of spliceosomal complexes. Also known as: snRNP U11, 12S U11 snRNP